{
  "gene_symbol": "HHAT",
  "gene": "UniProtKB:Q5VTY9",
  "term_id": "GO:0016409",
  "term_label": "palmitoyltransferase activity",
  "gene_name": "Protein-cysteine N-palmitoyltransferase HHAT"
}